{
  "gene_symbol": "PTMA",
  "gene": "UniProtKB:P06454",
  "term_label": "histone binding",
  "gene_name": "Prothymosin alpha",
  "term_id": "GO:0042393"
}